{
  "gene_name": "Zinc finger protein 776",
  "gene": "UniProtKB:Q68DI1",
  "term_label": "nucleus",
  "gene_symbol": "ZNF776",
  "term_id": "GO:0005634"
}